isogloboside biosynthetic process [GO:1990387] (biological process) References: PMID:35536927 Definition: The chemical reactions and pathways resulting in the formation of isogobliosides that begins with the synthesis of a tetrasaccharide core GalNAc-beta-1,3Gal-alpha-1,3Gal-beta-1,4Glc-ceramide. This core can be further elongated with the sequential addition of various carbohydrate units. Relationships: is a type of glycosphingolipid biosynthetic process [GO:0006688]; is a type of GO:0046513 Also known as: isoglobo-series glycosphingolipid biosynthesis